regulation of neuron projection regeneration [GO:0070570] (biological process) Subtypes: regulation of axon regeneration [GO:0048679], negative regulation of neuron projection regeneration [GO:0070571], positive regulation of neuron projection regeneration [GO:0070572] Relationships: is a type of regulation of neuron projection development [GO:0010975]; is a type of GO:0050793; is a type of GO:0080135; regulates GO:0031102 Sources: GOC:mah Definition: Any process that modulates the rate, frequency or extent of neuron projection regeneration, the regrowth of neuronal processes such as axons or dendrites following their loss or damage.